{
  "gene_symbol": "HLA-DOB",
  "term_id": "GO:0050870",
  "gene": "UniProtKB:P13765",
  "term_label": "positive regulation of T cell activation",
  "gene_name": "HLA class II histocompatibility antigen, DO beta chain"
}